Notch signaling pathway involved in regulation of secondary heart field cardioblast proliferation [GO:0003270] (biological process) Definition: The series of molecular signals initiated by binding of an extracellular ligand to a Notch receptor on the surface of the target cell contributing to the modulation of the frequency, rate or extent of cardioblast proliferation in the secondary heart field. A cardioblast is a cardiac precursor cell. It is a cell that has been committed to a cardiac fate, but will undergo more cell division rather than terminally differentiating. Also known as: Notch signalling pathway involved in regulation of secondary heart field cardioblast proliferation, Notch signaling pathway involved in regulation of second heart field cardioblast proliferation Sources: GOC:mtg_heart Relationships: is a type of Notch signaling involved in heart development [GO:0061314]; is part of regulation of secondary heart field cardioblast proliferation [GO:0003266]